{
  "gene": "UniProtKB:P10253",
  "gene_name": "Lysosomal alpha-glucosidase",
  "term_id": "GO:0005980",
  "gene_symbol": "GAA",
  "term_label": "glycogen catabolic process"
}